thioglucosidase complex [GO:0010169] (cellular component) Also known as: myrosinase complex Relationships: is a type of intracellular protein-containing complex [GO:0140535]; is a type of catalytic complex [GO:1902494] Definition: A large (200-800 kDa) multiprotein complex formed by 70-kDa and 5-kDa myrosinases, myrosinase- binding proteins (MBPs), MBP-related proteins and myrosinase-associated proteins. The complex has been identified in Brassica napus seeds. References: PMID:10682349